regulation of Golgi lumen acidification [GO:1905526] (biological process) References: PMID:23447592 Sources: GOC:TermGenie, GOC:dph, GO_REF:0000058 Relationships: is a type of GO:0032847; RO_0002211 GO:0061795 Definition: Any process that modulates the frequency, rate or extent of Golgi lumen acidification. Subtypes: negative regulation of Golgi lumen acidification [GO:1905527], positive regulation of Golgi lumen acidification [GO:1905528]